{
  "term_id": "GO:0005737",
  "gene_symbol": "CDC42EP3",
  "gene": "UniProtKB:Q9UKI2",
  "term_label": "cytoplasm",
  "gene_name": "Cdc42 effector protein 3"
}